{
  "term_id": "GO:0005788",
  "gene_symbol": "TOR1A",
  "gene_name": "Torsin-1A",
  "gene": "UniProtKB:O14656",
  "term_label": "endoplasmic reticulum lumen"
}